{
  "gene_symbol": "ISL2",
  "gene": "UniProtKB:Q96A47",
  "gene_name": "Insulin gene enhancer protein ISL-2",
  "term_id": "GO:0007409",
  "term_label": "axonogenesis"
}